somatic diversification of DSCAM-based immune receptors [GO:0002201] (biological process) Definition: The somatic process that results in the generation of sequence diversity of the DSCAM-based immune receptors of insects. References: PMID:16261174 Sources: GOC:add Note: Note that this type of immune receptor may not be limited to insects. Relationships: is a type of GO:0002200